{
  "gene": "UniProtKB:Q9H3K6",
  "gene_name": "BolA-like protein 2",
  "term_id": "GO:0005829",
  "term_label": "cytosol",
  "gene_symbol": "BOLA2"
}